{
  "gene_name": "E3 ubiquitin-protein ligase RNF185",
  "gene": "UniProtKB:Q96GF1",
  "term_label": "ubiquitin protein ligase activity",
  "term_id": "GO:0061630",
  "gene_symbol": "RNF185"
}